{
  "term_label": "nucleus",
  "gene_symbol": "FHL2",
  "term_id": "GO:0005634",
  "gene_name": "Four and a half LIM domains protein 2",
  "gene": "UniProtKB:Q14192"
}